{
  "term_id": "GO:0005737",
  "term_label": "cytoplasm",
  "gene": "UniProtKB:O75582",
  "gene_name": "Ribosomal protein S6 kinase alpha-5",
  "gene_symbol": "RPS6KA5"
}